radial spoke assembly [GO:0062177] (biological process) Relationships: is a type of protein-containing complex assembly [GO:0065003]; is part of GO:0035082 References: PMID:21613541, PMID:21692193, PMID:24124175, PMID:27940518, PMID:8408197 Definition: The aggregation, arrangement and bonding together of a set of components to form the radial spoke, a protein complex that links the outer microtubule doublet of the ciliary or flagellum axoneme with the sheath that surrounds the central pair of microtubules.